{
  "term_label": "galactose catabolic process via UDP-galactose, Leloir pathway",
  "term_id": "GO:0033499",
  "gene": "UniProtKB:Q14376",
  "gene_symbol": "GALE",
  "gene_name": "UDP-glucose 4-epimerase"
}